{
  "term_id": "UNKNOWN:0001",
  "gene_name": "Protein FAM74A1",
  "gene": "UniProtKB:Q5RGS3",
  "term_label": "Unknown molecular function",
  "gene_symbol": "FAM74A1"
}